{
  "gene_symbol": "NDUFAF1",
  "gene_name": "Complex I intermediate-associated protein 30, mitochondrial",
  "term_label": "mitochondrion",
  "term_id": "GO:0005739",
  "gene": "UniProtKB:Q9Y375"
}